{
  "gene_name": "Rap guanine nucleotide exchange factor-like 1",
  "gene": "UniProtKB:Q9UHV5",
  "term_label": "guanyl-nucleotide exchange factor activity",
  "term_id": "GO:0005085",
  "gene_symbol": "RAPGEFL1"
}